5,6-dimethylbenzimidazole synthase activity [GO:0102919] (molecular function) Relationships: is a type of GO:0016702 Sources: EC:1.13.11.79 Definition: Catalysis of the reaction: FMNH2 + O2 = 5,6-dimethylbenzimidazole + D-erythrose 4-phosphate + dialuric acid.